{
  "term_label": "Unknown molecular function",
  "gene": "UniProtKB:A0A576",
  "term_id": "UNKNOWN:0001",
  "gene_name": "T cell receptor beta variable 3-1",
  "gene_symbol": "TRBV3-1"
}